{
  "gene_name": "Protein-glutamine gamma-glutamyltransferase K",
  "term_id": "UNKNOWN:0003",
  "gene": "UniProtKB:P22735",
  "gene_symbol": "TGM1",
  "term_label": "Unknown cellular component"
}